{
  "gene_symbol": "SERTAD2",
  "gene_name": "SERTA domain-containing protein 2",
  "gene": "UniProtKB:Q14140",
  "term_label": "Unknown biological process",
  "term_id": "UNKNOWN:0002"
}